interleukin-1 receptor activity [GO:0004908] (molecular function) Also known as: IL-1 receptor activity, IL-1R Definition: Combining with interleukin-1 to initiate a change in cell activity. Interleukin-1 is produced mainly by activated macrophages and is involved in the inflammatory response. Sources: GOC:jl Relationships: is a type of cytokine receptor activity [GO:0004896]; has part GO:0019966 Subtypes: interleukin-1, type I, activating receptor activity [GO:0004909], GO:0004910